DNA repair-dependent chromatin remodeling [GO:0140861] (biological process) Relationships: is a type of chromatin remodeling [GO:0006338]; is part of DNA damage response [GO:0006974] Definition: A chromatin remodeling process that allows DNA repair enzyme to access genomic DNA and repair DNA lesions. References: PMID:15528408, PMID:28053344, PMID:29095668, PMID:35689883 Also known as: DNA damage-dependent chromatin remodelling